{
  "term_label": "Unknown biological process",
  "gene_symbol": "PACRG",
  "term_id": "UNKNOWN:0002",
  "gene_name": "Parkin coregulated gene protein",
  "gene": "UniProtKB:Q96M98"
}